positive regulation of monopolar cell growth [GO:0051515] (biological process) Sources: GOC:ai Subtypes: activation of monopolar cell growth [GO:0051522] Definition: Any process that activates or increases the frequency, rate or extent of monopolar cell growth, polarized growth from one end of a cell. Relationships: is a type of GO:0051512; is a type of regulation of monopolar cell growth [GO:0051513]; positively regulates monopolar cell growth [GO:0042814] Also known as: up regulation of monopolar cell growth, up-regulation of monopolar cell growth, upregulation of monopolar cell growth, stimulation of monopolar cell growth